{
  "gene": "UniProtKB:A2RUC4",
  "term_id": "GO:0000049",
  "gene_name": "tRNA wybutosine-synthesizing protein 5",
  "gene_symbol": "TYW5",
  "term_label": "tRNA binding"
}